{
  "gene": "UniProtKB:Q9NRM1",
  "gene_symbol": "ENAM",
  "gene_name": "Enamelin",
  "term_id": "GO:0036305",
  "term_label": "ameloblast differentiation"
}